terpenoid biosynthetic process, mevalonate-independent [GO:0051483] (BP) Definition: The chemical reactions and pathways resulting in the formation of terpenoids, independent of mevalonate. Isopentenyl diphosphate (IPP) is the fundamental unit in terpenoid biosynthesis, and in mevalonate-independent biosynthesis, it is produced from pyruvate and glyceraldehyde 3-phosphate via intermediates including 1-deoxy-D-xylulose 5-phosphate. Sources: GOC:ai Also known as: mevalonate-independent terpenoid biosynthesis, mevalonate-independent terpenoid biosynthetic process, terpenoid anabolism, mevalonate-independent, terpenoid formation, mevalonate-independent, terpenoid synthesis, mevalonate-independent, mevalonate-independent terpene biosynthesis, mevalonate-independent terpene biosynthetic process, terpene biosynthesis, mevalonate-independent, terpene biosynthetic process, mevalonate-independent Relationships: is a type of terpenoid biosynthetic process [GO:0016114]